{
  "term_label": "GTPase activity",
  "gene_name": "Rho-related BTB domain-containing protein 2",
  "gene": "UniProtKB:Q9BYZ6",
  "gene_symbol": "RHOBTB2",
  "term_id": "GO:0003924"
}